{
  "term_id": "UNKNOWN:0002",
  "gene_name": "Small integral membrane protein 47",
  "gene": "UniProtKB:D0EPY3",
  "gene_symbol": "SMIM47",
  "term_label": "Unknown biological process"
}